branch elongation involved in salivary gland morphogenesis [GO:0060667] (biological process) Definition: The differential growth of the salivary branches along their axis, resulting in the growth of a branch. Sources: GOC:dph Relationships: is a type of GO:0060602; is part of branching involved in salivary gland morphogenesis [GO:0060445]